cinnamic acid ester catabolic process [GO:0046282] (biological process) Sources: GOC:ai Definition: The chemical reactions and pathways resulting in the breakdown of ester derivatives of cinnamic acid, phenylpropenoic acid. Also known as: cinnamic acid ester breakdown, cinnamic acid ester catabolism, cinnamic acid ester degradation Relationships: is a type of cinnamic acid ester metabolic process [GO:0009801]; is a type of phenylpropanoid catabolic process [GO:0046271]; is a type of olefinic compound catabolic process [GO:0120256]